{
  "term_label": "prenyltransferase activity",
  "gene_name": "All trans-polyprenyl-diphosphate synthase PDSS1",
  "term_id": "GO:0004659",
  "gene": "UniProtKB:Q5T2R2",
  "gene_symbol": "PDSS1"
}